{
  "term_id": "GO:0097001",
  "term_label": "ceramide binding",
  "gene": "UniProtKB:Q9UBY8",
  "gene_symbol": "CLN8",
  "gene_name": "Protein CLN8"
}